glycerol ether biosynthetic process [GO:0046504] (biological process) Relationships: is a type of ether biosynthetic process [GO:1901503] Subtypes: ether lipid biosynthetic process [GO:0008611] Also known as: glycerol ether anabolism, glycerol ether biosynthesis, glycerol ether formation, glycerol ether synthesis Sources: GOC:ai Definition: The chemical reactions and pathways resulting in the formation of glycerol ethers, any anhydride formed between two organic hydroxy compounds, one of which is glycerol.